{
  "term_label": "Unknown molecular function",
  "gene_name": "General transcription factor 3C polypeptide 3",
  "term_id": "UNKNOWN:0001",
  "gene_symbol": "GTF3C3",
  "gene": "UniProtKB:Q9Y5Q9"
}